{
  "term_label": "regulation of microtubule cytoskeleton organization",
  "term_id": "GO:0070507",
  "gene_name": "Microtubule-associated protein 6",
  "gene": "UniProtKB:Q96JE9",
  "gene_symbol": "MAP6"
}